{
  "gene_name": "Desmoglein-4",
  "term_id": "GO:0030057",
  "gene": "UniProtKB:Q86SJ6",
  "term_label": "desmosome",
  "gene_symbol": "DSG4"
}